{
  "gene": "UniProtKB:O43781",
  "term_id": "GO:0004674",
  "term_label": "protein serine/threonine kinase activity",
  "gene_symbol": "DYRK3",
  "gene_name": "Dual specificity tyrosine-phosphorylation-regulated kinase 3"
}